{
  "gene": "UniProtKB:O00408",
  "term_id": "GO:0005759",
  "gene_name": "cGMP-dependent 3',5'-cyclic phosphodiesterase",
  "term_label": "mitochondrial matrix",
  "gene_symbol": "PDE2A"
}